{
  "gene_symbol": "ACSM4",
  "gene": "UniProtKB:P0C7M7",
  "term_id": "GO:0006637",
  "gene_name": "Acyl-coenzyme A synthetase ACSM4, mitochondrial",
  "term_label": "acyl-CoA metabolic process"
}